{
  "gene_name": "Developmental pluripotency-associated protein 2",
  "gene_symbol": "DPPA2",
  "gene": "UniProtKB:Q7Z7J5",
  "term_id": "GO:0003682",
  "term_label": "chromatin binding"
}